{
  "gene": "UniProtKB:Q8IWZ3",
  "term_label": "Unknown molecular function",
  "gene_name": "Ankyrin repeat and KH domain-containing protein 1",
  "term_id": "UNKNOWN:0001",
  "gene_symbol": "ANKHD1"
}